{
  "gene_name": "Transcription factor SOX-4",
  "gene_symbol": "SOX4",
  "term_label": "negative regulation of transcription by RNA polymerase II",
  "term_id": "GO:0000122",
  "gene": "UniProtKB:Q06945"
}